{
  "term_id": "UNKNOWN:0001",
  "gene_name": "Ran-binding protein 3",
  "term_label": "Unknown molecular function",
  "gene": "UniProtKB:Q9H6Z4",
  "gene_symbol": "RANBP3"
}